{
  "term_id": "GO:0006094",
  "term_label": "gluconeogenesis",
  "gene_symbol": "G6PC3",
  "gene": "UniProtKB:Q9BUM1",
  "gene_name": "Glucose-6-phosphatase 3"
}